fat body development [GO:0007503] (biological process) Sources: ISBN:0582227089 Subtypes: larval fat body development [GO:0007504], adult fat body development [GO:0007505] Definition: The process whose specific outcome is the progression of the fat body over time, from its formation to the mature structure. A fat body is an insect gland dorsal to the insect gut, with a function analogous to that of the vertebrate liver. It is a storage organ for fats, glycogen and protein and is a major site of intermediary metabolism. Relationships: is a type of animal organ development [GO:0048513]